synaptobrevin 2-SNAP-25-syntaxin-1a-complexin I complex [GO:0070032] (cellular component) Relationships: is a type of SNARE complex [GO:0031201] Definition: A SNARE complex that contains synaptobrevin 2 (VAMP2), SNAP-25, syntaxin 1a, and complexin I (or orthologs thereof). Also known as: SNARE complex (Vamp2, Snap25, Stx1a, Cplx1), Vamp2-Snap25-Stx1a-Cplx1 complex References: PMID:7553862